{
  "term_label": "DNA-binding transcription factor activity, RNA polymerase II-specific",
  "term_id": "GO:0000981",
  "gene": "UniProtKB:P0CI00",
  "gene_symbol": "ZNF705B",
  "gene_name": "Putative zinc finger protein 705B"
}